{
  "term_label": "Swi5-Sfr1 complex",
  "gene_name": "DNA repair protein SWI5 homolog",
  "gene": "UniProtKB:Q1ZZU3",
  "gene_symbol": "SWI5",
  "term_id": "GO:0032798"
}